bubble DNA binding [GO:0000405] (molecular function) Definition: Binding to DNA segment that contains a bubble. A bubble occurs when DNA contains a region of unpaired, single-stranded DNA flanked on both sides by regions of paired, double-stranded DNA. References: PMID:16781730 Sources: GOC:elh, GOC:vw Relationships: is a type of DNA secondary structure binding [GO:0000217]